carbohydrate phosphatase activity [GO:0019203] (molecular function) Relationships: is a type of phosphatase activity [GO:0016791] Subtypes: sugar-phosphatase activity [GO:0050308] Sources: GOC:mah Definition: Catalysis of the reaction: carbohydrate phosphate + H2O = carbohydrate + phosphate.